trichome morphogenesis [GO:0010090] (biological process) Relationships: is a type of cell morphogenesis [GO:0000902]; is part of GO:0010026; is part of GO:0090626 Regulation: regulated by regulation of trichome morphogenesis [GO:2000039] Sources: GOC:mtg_sensu, GOC:tair_curators Also known as: trichome cell morphogenesis during differentiation Definition: The process in which the structures of a hair cell (trichome) cell are generated and organized. This process occurs while the initially relatively unspecialized epidermal cell is acquiring the specialized features of a hair cell. An example of this process is found in Arabidopsis thaliana.